collagen type V trimer [GO:0005588] (cellular component) Relationships: is a type of fibrillar collagen trimer [GO:0005583] Definition: A collagen heterotrimer containing type V alpha chains; [alpha1(V)]2alpha2(V) and alpha1(V)alpha2(V)alpha3(V) trimers have been observed; type V collagen triple helices associate to form fibrils. References: PMID:21421911